acinar cell differentiation [GO:0090425] (biological process) Definition: The epithelial cell differentiation process in which a relatively unspecialized cell acquires specialized features of an acinar cell, a secretory cell that is grouped together with other cells of the same type to form grape-shaped clusters known as acini. Relationships: is_a GO:0002067 Subtypes: acinar cell differentiation involved in salivary gland development [GO:0060704], GO:1903680 Sources: GOC:dph, GOC:tb